{
  "gene_name": "Protein Wnt-10b",
  "gene_symbol": "WNT10B",
  "term_id": "GO:0005125",
  "term_label": "cytokine activity",
  "gene": "UniProtKB:O00744"
}